{
  "gene_name": "Ras-related protein Rab-44",
  "term_label": "GTP binding",
  "gene_symbol": "RAB44",
  "term_id": "GO:0005525",
  "gene": "UniProtKB:Q7Z6P3"
}